{
  "term_id": "GO:0006357",
  "term_label": "regulation of transcription by RNA polymerase II",
  "gene": "UniProtKB:Q9P0T4",
  "gene_name": "Zinc finger protein 581",
  "gene_symbol": "ZNF581"
}